{
  "term_id": "GO:0030027",
  "term_label": "lamellipodium",
  "gene_symbol": "CORO1C",
  "gene": "UniProtKB:Q9ULV4",
  "gene_name": "Coronin-1C"
}